{
  "gene_name": "Partitioning defective 6 homolog beta",
  "term_id": "UNKNOWN:0001",
  "term_label": "Unknown molecular function",
  "gene": "UniProtKB:Q9BYG5",
  "gene_symbol": "PARD6B"
}